{
  "gene_name": "Upstream-binding protein 1",
  "term_id": "GO:0006357",
  "gene_symbol": "UBP1",
  "term_label": "regulation of transcription by RNA polymerase II",
  "gene": "UniProtKB:Q9NZI7"
}